{
  "gene": "UniProtKB:D6REC4",
  "term_label": "Unknown molecular function",
  "gene_name": "Cilia- and flagella-associated protein 99",
  "gene_symbol": "CFAP99",
  "term_id": "UNKNOWN:0001"
}